spindle pole centrosome [GO:0031616] (cellular component) Definition: A centrosome from which one pole of a mitotic or meiotic spindle is organized. Sources: GOC:mah Relationships: is a type of centrosome [GO:0005813]; is part of spindle pole [GO:0000922]